{
  "gene_symbol": "ZNF225",
  "gene": "UniProtKB:Q9UK10",
  "term_id": "GO:0005634",
  "term_label": "nucleus",
  "gene_name": "Zinc finger protein 225"
}